perianth development [GO:0090428] (biological process) Sources: GOC:tb, PO:0009058 Relationships: is a type of floral whorl development [GO:0048438] Definition: The process whose specific outcome is the progression of the perianth over time, from its formation to the mature structure. The perianth is a collective phyllome structure composed of two or more petals, sepals, or tepals.